{
  "gene_symbol": "CDH4",
  "gene_name": "Cadherin-4",
  "gene": "UniProtKB:P55283",
  "term_id": "GO:0005912",
  "term_label": "adherens junction"
}